{
  "gene": "UniProtKB:Q08722",
  "gene_symbol": "CD47",
  "term_id": "GO:0050766",
  "term_label": "positive regulation of phagocytosis",
  "gene_name": "Leukocyte surface antigen CD47"
}